{
  "gene": "UniProtKB:Q6PL45",
  "term_id": "UNKNOWN:0001",
  "term_label": "Unknown molecular function",
  "gene_symbol": "BRICD5",
  "gene_name": "BRICHOS domain-containing protein 5"
}